tRNA decay [GO:0016078] (biological process) Definition: The chemical reactions and pathways resulting in the breakdown of tRNA, transfer RNA, a class of relatively small RNA molecules responsible for mediating the insertion of amino acids into the sequence of nascent polypeptide chains during protein synthesis. Regulation: regulated by regulation of tRNA catabolic process [GO:1902370]; negatively regulated by negative regulation of tRNA catabolic process [GO:1902371]; positively regulated by GO:1902372 Relationships: is a type of tRNA metabolic process [GO:0006399]; is a type of GO:0006401 Sources: GOC:ai Also known as: tRNA breakdown, tRNA catabolic process, tRNA catabolism, tRNA degradation Subtypes: tRNA surveillance [GO:0106354]